{
  "term_id": "UNKNOWN:0002",
  "gene_symbol": "UNQ9370_PRO34162",
  "gene_name": "Putative uncharacterized protein UNQ9370_PRO34162",
  "gene": "UniProtKB:Q6UXP9",
  "term_label": "Unknown biological process"
}